{
  "term_id": "GO:0005634",
  "term_label": "nucleus",
  "gene_name": "Serine_threonine-protein phosphatase 2A activator",
  "gene_symbol": "PTPA",
  "gene": "UniProtKB:Q15257"
}